pyruvate synthase activity [GO:0019164] (molecular function) Sources: KEGG_REACTION:R01196 Definition: Catalysis of the reaction: pyruvate + CoA + 2 oxidized ferredoxin = acetyl-CoA + CO2 + 2 reduced ferredoxin + 2 H+. Relationships: is a type of oxidoreductase activity, acting on the aldehyde or oxo group of donors, iron-sulfur protein as acceptor [GO:0016625]; is part of pyruvate decarboxylation to acetyl-CoA [GO:0006086] Also known as: PFOR, pyruvate-ferredoxin reductase activity, pyruvate oxidoreductase activity, pyruvate synthetase activity, pyruvate:ferredoxin 2-oxidoreductase (CoA-acetylating), pyruvate:ferredoxin oxidoreductase activity, pyruvic-ferredoxin oxidoreductase activity